{
  "term_label": "RNA polymerase II cis-regulatory region sequence-specific DNA binding",
  "gene_name": "Krueppel-like factor 1",
  "gene": "UniProtKB:Q13351",
  "term_id": "GO:0000978",
  "gene_symbol": "KLF1"
}